{
  "gene": "UniProtKB:P62917",
  "gene_symbol": "RPL8",
  "term_id": "GO:0003735",
  "term_label": "structural constituent of ribosome",
  "gene_name": "Large ribosomal subunit protein uL2"
}